{
  "gene_name": "Leucine-rich repeat-containing protein 56",
  "term_label": "Unknown cellular component",
  "gene_symbol": "LRRC56",
  "term_id": "UNKNOWN:0003",
  "gene": "UniProtKB:Q8IYG6"
}